{
  "term_label": "Unknown molecular function",
  "gene_symbol": "CCDC30",
  "term_id": "UNKNOWN:0001",
  "gene_name": "Coiled-coil domain-containing protein 30",
  "gene": "UniProtKB:Q5VVM6"
}